{
  "gene": "UniProtKB:Q8N4C6",
  "gene_symbol": "NIN",
  "term_label": "mitotic spindle pole",
  "term_id": "GO:0097431",
  "gene_name": "Ninein"
}